palisade mesophyll development [GO:1903866] (biological process) References: PMID:24663344 Sources: GOC:TermGenie, GO_REF:0000080 Also known as: palisade parenchyma development Relationships: is_a anatomical structure development [GO:0048856] Definition: The process whose specific outcome is the progression of a palisade mesophyll over time, from its formation to the mature structure.